{
  "gene_symbol": "PRKDC",
  "gene": "UniProtKB:P78527",
  "term_id": "GO:0005634",
  "gene_name": "DNA-dependent protein kinase catalytic subunit",
  "term_label": "nucleus"
}